{
  "gene": "UniProtKB:P10826",
  "gene_name": "Retinoic acid receptor beta",
  "term_id": "GO:0005634",
  "term_label": "nucleus",
  "gene_symbol": "RARB"
}